{
  "gene_name": "Protein SPT2 homolog",
  "gene": "UniProtKB:Q68D10",
  "term_id": "GO:0003677",
  "term_label": "DNA binding",
  "gene_symbol": "SPTY2D1"
}